{
  "term_label": "7S RNA binding",
  "gene_symbol": "SRP54",
  "gene_name": "Signal recognition particle subunit SRP54",
  "term_id": "GO:0008312",
  "gene": "UniProtKB:P61011"
}